{
  "gene_name": "Dynein axonemal assembly factor 4",
  "term_label": "epithelial cilium movement involved in extracellular fluid movement",
  "term_id": "GO:0003351",
  "gene": "UniProtKB:Q8WXU2",
  "gene_symbol": "DNAAF4"
}